{
  "term_label": "nucleoplasm",
  "gene": "UniProtKB:Q8TEC5",
  "term_id": "GO:0005654",
  "gene_symbol": "SH3RF2",
  "gene_name": "E3 ubiquitin-protein ligase SH3RF2"
}